{
  "gene": "UniProtKB:O14519",
  "gene_name": "Cyclin-dependent kinase 2-associated protein 1",
  "term_label": "Unknown molecular function",
  "gene_symbol": "CDK2AP1",
  "term_id": "UNKNOWN:0001"
}